{
  "gene": "UniProtKB:Q07912",
  "term_id": "UNKNOWN:0002",
  "gene_symbol": "TNK2",
  "gene_name": "Activated CDC42 kinase 1",
  "term_label": "Unknown biological process"
}